regulation of protein localization to non-growing cell tip [GO:0062107] (biological process) Subtypes: negative regulation of protein localization to non-growing cell tip [GO:0062108] Definition: Any process that modulates the frequency, rate or extent of protein localization to a non-growing cell tip. Relationships: is a type of GO:1903066; regulates protein localization to non-growing cell tip [GO:1902487] References: PMID:18328707